{
  "gene_name": "Protein FAM13A",
  "term_id": "UNKNOWN:0001",
  "gene": "UniProtKB:O94988",
  "gene_symbol": "FAM13A",
  "term_label": "Unknown molecular function"
}